{
  "term_id": "GO:0046085",
  "term_label": "adenosine metabolic process",
  "gene": "UniProtKB:P49902",
  "gene_symbol": "NT5C2",
  "gene_name": "Cytosolic purine 5'-nucleotidase"
}